zeaxanthin epoxidase activity [GO:0052662] (molecular function) Relationships: is a type of oxidoreductase activity, acting on paired donors, with incorporation or reduction of molecular oxygen, reduced iron-sulfur protein as one donor, and incorporation of one atom of oxygen [GO:0016713] Definition: Catalysis of the reaction: all-trans-zeaxanthin + 4 H+ + 2 O2 + 4 reduced [2Fe-2S]-[ferredoxin] = all-trans-violaxanthin + 2 H2O + 4 oxidized [2Fe-2S]-[ferredoxin]. Sources: RHEA:32443 Also known as: antheraxanthin epoxidase activity, zea-epoxidase activity, zeaxanthin epoxidase [overall] activity